{
  "term_id": "GO:0006357",
  "gene_symbol": "TCF7L2",
  "gene": "UniProtKB:Q9NQB0",
  "term_label": "regulation of transcription by RNA polymerase II",
  "gene_name": "Transcription factor 7-like 2"
}